{
  "gene_symbol": "SPINT2",
  "term_label": "epithelial cell morphogenesis",
  "term_id": "GO:0003382",
  "gene_name": "Kunitz-type protease inhibitor 2",
  "gene": "UniProtKB:O43291"
}